{
  "gene_symbol": "C1D",
  "gene_name": "Nuclear nucleic acid-binding protein C1D",
  "term_id": "GO:0000178",
  "term_label": "exosome (RNase complex)",
  "gene": "UniProtKB:Q13901"
}